{
  "gene_name": "Partitioning defective 3 homolog",
  "term_id": "GO:0005912",
  "term_label": "adherens junction",
  "gene": "UniProtKB:Q8TEW0",
  "gene_symbol": "PARD3"
}